{
  "term_id": "UNKNOWN:0003",
  "gene_name": "Forkhead box protein N1",
  "term_label": "Unknown cellular component",
  "gene_symbol": "FOXN1",
  "gene": "UniProtKB:O15353"
}